termination of RNA polymerase II transcription [GO:0006369] (biological process) Relationships: is a type of DNA-templated transcription termination [GO:0006353]; is part of transcription by RNA polymerase II [GO:0006366] References: PMID:27371117 Sources: GOC:mah, GOC:txnOH Subtypes: termination of RNA polymerase II transcription, poly(A)-coupled [GO:0030846], termination of RNA polymerase II transcription, exosome-dependent [GO:0030847] Also known as: RNA 3'-end formation by RNA polymerase II, RNA polymerase II transcription termination, transcription termination from Pol II promoter, transcription termination from RNA polymerase II promoter, RNA polymerase II transcription termination factor activity Regulation: negatively regulated by GO:0120191; regulated by regulation of termination of RNA polymerase II transcription [GO:1904594]; positively regulated by positive regulation of termination of RNA polymerase II transcription [GO:1904595] Definition: A transcription termination process that completes the production of a primary RNA polymerase II transcript.